{
  "gene": "UniProtKB:Q96DB5",
  "gene_name": "Regulator of microtubule dynamics protein 1",
  "term_id": "GO:0097431",
  "term_label": "mitotic spindle pole",
  "gene_symbol": "RMDN1"
}